{
  "gene_name": "Zinc finger CCHC domain-containing protein 7",
  "gene_symbol": "ZCCHC7",
  "gene": "UniProtKB:Q8N3Z6",
  "term_id": "GO:0071038",
  "term_label": "TRAMP-dependent tRNA surveillance pathway"
}